{
  "term_id": "UNKNOWN:0001",
  "term_label": "Unknown molecular function",
  "gene_name": "Spermatogenesis-associated protein 31A6",
  "gene": "UniProtKB:Q5VVP1",
  "gene_symbol": "SPATA31A6"
}